{
  "term_label": "Unknown molecular function",
  "gene_symbol": "CMC4",
  "gene_name": "Cx9C motif-containing protein 4",
  "gene": "UniProtKB:P56277",
  "term_id": "UNKNOWN:0001"
}